{
  "gene": "UniProtKB:Q96SI1",
  "gene_name": "BTB_POZ domain-containing protein KCTD15",
  "term_label": "Unknown cellular component",
  "term_id": "UNKNOWN:0003",
  "gene_symbol": "KCTD15"
}